{
  "gene_symbol": "ZFP82",
  "term_label": "regulation of transcription by RNA polymerase II",
  "gene_name": "Zinc finger protein 82 homolog",
  "gene": "UniProtKB:Q8N141",
  "term_id": "GO:0006357"
}